{
  "gene": "UniProtKB:Q12926",
  "term_label": "Unknown cellular component",
  "gene_symbol": "ELAVL2",
  "term_id": "UNKNOWN:0003",
  "gene_name": "ELAV-like protein 2"
}